CD4-positive, alpha-beta intraepithelial T cell differentiation [GO:0002301] (biological process) Note: Note that immunologists typically use the word 'development' to refer to cells of B or T cell lineages undergoing the process that GO describes as 'cell differentiation'. Sources: GOC:add, ISBN:0781735149 Definition: The process in which a precursor cell type acquires the specialized features of a CD4-positive, alpha-beta intraepithelial T cell. Intraepithelial T cells are found among epithelial cells in mucosal areas and have distinct phenotypes and developmental pathways. Also known as: CD4-positive, alpha-beta intraepithelial T lymphocyte differentiation, CD4-positive, alpha-beta intraepithelial T-cell differentiation, CD4-positive, alpha-beta intraepithelial T-lymphocyte differentiation, CD4-positive, alpha-beta intraepithelial T cell development Relationships: is_a alpha-beta intraepithelial T cell differentiation [GO:0002299]; is a type of CD4-positive, alpha-beta T cell differentiation [GO:0043367]